{
  "gene_name": "Ciliary neurotrophic factor receptor subunit alpha",
  "gene": "UniProtKB:P26992",
  "term_id": "GO:0070110",
  "gene_symbol": "CNTFR",
  "term_label": "ciliary neurotrophic factor receptor complex"
}